{
  "gene_symbol": "NKX6-1",
  "term_id": "GO:0030154",
  "gene": "UniProtKB:P78426",
  "gene_name": "Homeobox protein Nkx-6.1",
  "term_label": "cell differentiation"
}